{
  "term_id": "GO:0009986",
  "gene": "UniProtKB:Q7RTW8",
  "gene_symbol": "OTOA",
  "gene_name": "Otoancorin",
  "term_label": "cell surface"
}